{
  "gene": "UniProtKB:O00203",
  "term_id": "GO:0048490",
  "gene_symbol": "AP3B1",
  "gene_name": "AP-3 complex subunit beta-1",
  "term_label": "anterograde synaptic vesicle transport"
}